{
  "gene_name": "Protein CD300H",
  "gene": "UniProtKB:A0A0K2S4Q6",
  "gene_symbol": "CD300H",
  "term_id": "GO:0045088",
  "term_label": "regulation of innate immune response"
}